{
  "gene": "UniProtKB:Q96LD4",
  "gene_symbol": "TRIM47",
  "term_label": "Unknown molecular function",
  "gene_name": "E3 ubiquitin-protein ligase TRIM47",
  "term_id": "UNKNOWN:0001"
}